{
  "term_id": "UNKNOWN:0003",
  "gene_symbol": "BTBD8",
  "gene": "UniProtKB:Q5XKL5",
  "term_label": "Unknown cellular component",
  "gene_name": "BTB_POZ domain-containing protein 8"
}